protein-FAD linkage [GO:0018293] (biological process) Definition: The formation of a linkage between a protein amino acid and flavin-adenine dinucleotide (FAD). Sources: GOC:ai Relationships: is a type of GO:0036211